protein localization to cell tip [GO:1990151] (biological process) Regulation: regulated by regulation of protein localization to cell tip [GO:1903066]; negatively regulated by negative regulation of protein localization to cell tip [GO:1903067]; positively regulated by positive regulation of protein localization to cell tip [GO:1903068] Subtypes: protein transport along microtubule to cell tip [GO:0099117], protein localization to growing cell tip [GO:1902486], protein localization to non-growing cell tip [GO:1902487], protein localization to mating projection tip [GO:1903260], protein localization to plasma membrane of cell tip [GO:1903418], protein localization to cell cortex of cell tip [GO:1990896] References: PMID:22768263 Definition: A process in which a protein is transported to, or maintained in, a location at the cell tip. Relationships: is a type of GO:0008104 Also known as: protein localisation to cell tip